{
  "term_label": "cell surface",
  "gene_name": "Tumor necrosis factor ligand superfamily member 18",
  "term_id": "GO:0009986",
  "gene_symbol": "TNFSF18",
  "gene": "UniProtKB:Q9UNG2"
}